positive regulation of intestinal lipid absorption [GO:1904731] (biological process) References: PMID:18768481 Sources: GOC:TermGenie, GO_REF:0000058 Subtypes: positive regulation of intestinal cholesterol absorption [GO:0045797] Also known as: up regulation of intestinal lipid absorption, up-regulation of intestinal lipid absorption, upregulation of intestinal lipid absorption, activation of intestinal lipid absorption Relationships: is a type of GO:1904480; is a type of regulation of intestinal lipid absorption [GO:1904729]; positively regulates intestinal lipid absorption [GO:0098856] Definition: Any process that activates or increases the frequency, rate or extent of intestinal lipid absorption.